{
  "gene_name": "General transcription factor 3C polypeptide 1",
  "term_id": "GO:0006384",
  "gene": "UniProtKB:Q12789",
  "gene_symbol": "GTF3C1",
  "term_label": "transcription initiation at RNA polymerase III promoter"
}